uredinium development [GO:0075279] (biological process) Sources: GOC:pamgo_curators Regulation: regulated by regulation of uredinium development [GO:0075280]; positively regulated by positive regulation of uredinium development [GO:0075281]; negatively regulated by GO:0075282 Definition: The process that leads to the formation of a uredinium, a reddish, pustule-like structure formed by a rust fungus and consisting of uredospores. Relationships: is a type of GO:0075259 Also known as: development of uredium